{
  "gene": "UniProtKB:Q15847",
  "gene_symbol": "ADIRF",
  "term_id": "GO:0045600",
  "term_label": "positive regulation of fat cell differentiation",
  "gene_name": "Adipogenesis regulatory factor"
}